{
  "gene_symbol": "C2orf72",
  "term_label": "Unknown cellular component",
  "term_id": "UNKNOWN:0003",
  "gene": "UniProtKB:A6NCS6",
  "gene_name": "Uncharacterized protein C2orf72"
}